IDP metabolic process [GO:0046707] (biological process) Also known as: IDP metabolism Sources: GOC:ai Definition: The chemical reactions and pathways involving IDP, inosine 5'-diphosphate. Relationships: is a type of purine ribonucleotide metabolic process [GO:0009150]; is a type of purine ribonucleoside diphosphate metabolic process [GO:0009179] Subtypes: GO:0046708, IDP catabolic process [GO:0046709]